{
  "gene_name": "Transcription factor BTF3",
  "term_id": "UNKNOWN:0002",
  "term_label": "Unknown biological process",
  "gene": "UniProtKB:P20290",
  "gene_symbol": "BTF3"
}